{
  "gene": "UniProtKB:P42262",
  "gene_name": "Glutamate receptor 2",
  "gene_symbol": "GRIA2",
  "term_id": "GO:0035249",
  "term_label": "synaptic transmission, glutamatergic"
}